{
  "gene_symbol": "VPREB1",
  "gene_name": "Immunoglobulin iota chain",
  "term_id": "GO:0019814",
  "gene": "UniProtKB:P12018",
  "term_label": "immunoglobulin complex"
}